{
  "term_label": "histone binding",
  "gene_name": "YEATS domain-containing protein 4",
  "gene": "UniProtKB:O95619",
  "term_id": "GO:0042393",
  "gene_symbol": "YEATS4"
}